{
  "term_id": "GO:0070585",
  "gene_symbol": "RNF186",
  "term_label": "protein localization to mitochondrion",
  "gene": "UniProtKB:Q9NXI6",
  "gene_name": "E3 ubiquitin-protein ligase RNF186"
}